{
  "term_label": "endosome",
  "gene_name": "Ras-related protein Rab-3C",
  "gene_symbol": "RAB3C",
  "gene": "UniProtKB:Q96E17",
  "term_id": "GO:0005768"
}